{
  "gene": "UniProtKB:Q9H3Q1",
  "term_id": "GO:0031267",
  "term_label": "small GTPase binding",
  "gene_symbol": "CDC42EP4",
  "gene_name": "Cdc42 effector protein 4"
}